negative regulation of xylose catabolic process to ethanol [GO:1900516] (biological process) Relationships: is a type of GO:0009895; is a type of negative regulation of carbohydrate metabolic process [GO:0045912]; is a type of negative regulation of small molecule metabolic process [GO:0062014]; is_a GO:1900515; is a type of negative regulation of fermentation [GO:1901003]; negatively regulates D-xylose catabolic process to ethanol [GO:0044577] Also known as: down regulation of xylose catabolic process to ethanol, down regulation of xylose catabolism to ethanol, down-regulation of xylose catabolic process to ethanol, down-regulation of xylose catabolism to ethanol, downregulation of xylose catabolic process to ethanol, downregulation of xylose catabolism to ethanol, inhibition of xylose catabolism to ethanol, negative regulation of xylose catabolism to ethanol, inhibition of xylose catabolic process to ethanol Sources: GOC:TermGenie, GOC:mengo_curators Definition: Any process that stops, prevents or reduces the frequency, rate or extent of xylose catabolic process to ethanol.